positive regulation of ATP biosynthetic process [GO:2001171] (biological process) Relationships: is a type of positive regulation of purine nucleotide biosynthetic process [GO:1900373]; is_a positive regulation of ATP metabolic process [GO:1903580]; is a type of regulation of ATP biosynthetic process [GO:2001169]; RO_0002213 GO:0006754 Sources: GOC:obol Definition: Any process that activates or increases the frequency, rate or extent of ATP biosynthetic process. Also known as: positive regulation of ATP anabolism, positive regulation of ATP biosynthesis, positive regulation of ATP formation, positive regulation of ATP synthesis, positive regulation of ATP regeneration